organic cation transport [GO:0015695] (biological process) Sources: GOC:ai Definition: The directed movement of organic cations into, out of or within a cell, or between cells, by means of some agent such as a transporter or pore. Organic cations are atoms or small molecules with a positive charge which contain carbon in covalent linkage. Subtypes: S-adenosyl-L-methionine transport [GO:0015805], GO:0015816, L-leucine transport [GO:0015820], methionine transport [GO:0015821], GO:0015822, proline transport [GO:0015824], tryptophan transport [GO:0015827], tyrosine transport [GO:0015828], cadaverine transport [GO:0015839], methylammonium transport [GO:0015843], putrescine transport [GO:0015847], GO:0015848, acetylcholine transport [GO:0015870], choline transport [GO:0015871], norepinephrine transport [GO:0015874], GO:0015879, thiamine transport [GO:0015888], glycine betaine transport [GO:0031460], pyridoxal transport [GO:0031920], pyridoxamine transport [GO:0031922], alanine transport [GO:0032328], serine transport [GO:0032329], ethanolamine transport [GO:0034229], cysteine transport [GO:0042883], daunorubicin transport [GO:0043215], epinephrine transport [GO:0048241], histamine secretion, neurotransmission [GO:0061538], GO:0061539, sodium-dependent organic cation transport [GO:0070715], GO:0080121, L-histidine transmembrane transport [GO:0089709], GO:0097638, GO:0140484, L-phenylalanine import across plasma membrane [GO:0140925], 4-(trimethylammonio)butanoate transport [GO:1900751], GO:1900753, L-lysine transport [GO:1902022], GO:1902024, L-valine transmembrane transport [GO:1903785], L-glutamine import across plasma membrane [GO:1903803], L-isoleucine import across plasma membrane [GO:1903806], L-threonine import across plasma membrane [GO:1903807], GO:1903811, L-arginine transmembrane transport [GO:1903826], carcinine import across plasma membrane [GO:1905130], GO:1905329, GO:1990818, N-methylnicotinate transport [GO:2001143] Relationships: is a type of transport [GO:0006810]